D-tyrosine catabolic process [GO:1900829] (biological process) Relationships: is a type of aromatic amino acid family catabolic process [GO:0009074]; is_a D-amino acid catabolic process [GO:0019478] Also known as: D-tyrosine breakdown, D-tyrosine catabolism, D-tyrosine degradation Definition: The chemical reactions and pathways resulting in the breakdown of D-tyrosine. References: PMID:10766779 Sources: GOC:TermGenie